Slx1-Slx4 complex [GO:0033557] (cellular component) Definition: A heterodimeric protein complex that possesses an endonuclease activity that specifically cleaves certain types of branched DNA structures; because such structures often form during the replication ribosomal DNA (rDNA) repeats, the complex plays a role in the maintenance of rDNA. The subunits are known as Slx1 and Slx 4 in budding and fission yeasts, and are conserved in eukaryotes. References: PMID:14528010, PMID:16467377 Relationships: is a type of nuclear protein-containing complex [GO:0140513]; is part of nuclear chromosome [GO:0000228]